negative regulation of cyclin-dependent protein serine/threonine kinase activity [GO:0045736] (biological process) Relationships: is a type of regulation of cyclin-dependent protein serine/threonine kinase activity [GO:0000079]; is a type of negative regulation of cell cycle [GO:0045786]; is a type of GO:0071901; is a type of negative regulation of cyclin-dependent protein kinase activity [GO:1904030]; negatively regulates cyclin-dependent protein serine/threonine kinase activity [GO:0004693] Sources: GOC:go_curators, GOC:pr Definition: Any process that stops, prevents, or reduces the frequency, rate or extent of cyclin-dependent protein serine/threonine kinase activity.